protein poly-ADP-ribosylation [GO:0070212] (biological process) References: PMID:25043379 Sources: GOC:BHF, GOC:mah, GOC:rl Definition: The transfer of multiple ADP-ribose residues from NAD to a protein amino acid, forming a poly(ADP-ribose) chain. Relationships: is a type of post-translational protein modification [GO:0043687] Also known as: addition of poly-ADP-ribose to protein, poly(ADP-ribose) addition to protein, protein amino acid poly-ADP-ribosylation, protein poly(ADP-ribose) synthesis, protein poly(ADP-ribose) metabolism